{
  "gene_name": "Ras-related protein Rab-5B",
  "term_label": "endomembrane system",
  "gene_symbol": "RAB5B",
  "term_id": "GO:0012505",
  "gene": "UniProtKB:P61020"
}